positive regulation of membrane hyperpolarization [GO:1902632] (biological process) Relationships: is a type of GO:0048518; is a type of regulation of membrane hyperpolarization [GO:1902630]; positively regulates membrane hyperpolarization [GO:0060081] References: PMID:23223304 Sources: GOC:TermGenie, GO_REF:0000058 Definition: Any process that activates or increases the frequency, rate or extent of membrane hyperpolarization. Also known as: up regulation of membrane hyperpolarization, up-regulation of membrane hyperpolarization, upregulation of membrane hyperpolarization, activation of membrane hyperpolarization